lactate metabolic process [GO:0006089] (biological process) Definition: The chemical reactions and pathways involving lactate, the anion of lactic acid. Sources: ISBN:0198547684 Also known as: 2-hydroxypropanoate metabolic process, 2-hydroxypropanoate metabolism, alpha-hydroxypropionate metabolic process, alpha-hydroxypropionate metabolism, lactate metabolism Relationships: is a type of GO:0032787 Subtypes: lactate racemization [GO:0019247], lactate biosynthetic process [GO:0019249], L-threonine catabolic process to D-lactate [GO:0019517], glucose catabolic process to lactate [GO:0019659], mixed acid fermentation [GO:0019664], methylglyoxal catabolic process to lactate [GO:0061727], lactate catabolic process [GO:1903457]